{
  "term_label": "Unknown molecular function",
  "term_id": "UNKNOWN:0001",
  "gene": "UniProtKB:Q68D86",
  "gene_symbol": "CCDC102B",
  "gene_name": "Coiled-coil domain-containing protein 102B"
}